{
  "term_label": "BMP binding",
  "gene": "UniProtKB:Q9H2X0",
  "gene_symbol": "CHRD",
  "term_id": "GO:0036122",
  "gene_name": "Chordin"
}